motor neuron precursor migration involved in dorsal motor nucleus of vagus nerve formation [GO:0035765] (biological process) References: PMID:21262462 Sources: GOC:dgh Definition: The orderly movement of a motor neuron precursor cell that contributes to formation of the dorsal motor nucleus of the vagus nerve. Relationships: is_a cell migration in hindbrain [GO:0021535]; is part of dorsal motor nucleus of vagus nerve formation [GO:0035764]